cardiac endothelial to mesenchymal transition [GO:0140074] (biological process) Definition: A transition where a cardiac endothelial cell loses apical/basolateral polarity, severs intercellular adhesive junctions, degrades basement membrane components and becomes a migratory mesenchymal cell. Endocardial cells (specialized endothelial cells that line the heart) undergo EndMT, and give rise to mesenchymal cells necessary for proper heart development. EndMT, specifically generates valve progenitor cells that give rise to the mitral and tricuspid valves. EndMT also contributes to endocardial cushion formation, as well as to generation of cardiac fibroblasts and smooth muscle cells, but not cardiac myocytes. References: PMID:16162442, PMID:26053665 Sources: GOC:BHF, GOC:nc Also known as: EndMT, EndoMT Relationships: is a type of mesenchymal cell differentiation [GO:0048762] Regulation: regulated by regulation of cardiac endothelial to mesenchymal transition [GO:0061999]; positively regulated by positive regulation of cardiac endothelial to mesenchymal transition [GO:0062000]; negatively regulated by negative regulation of cardiac endothelial to mesenchymal transition [GO:0062001]